{
  "gene_name": "Protein phosphatase 1 regulatory subunit 35",
  "term_id": "GO:0045724",
  "gene_symbol": "PPP1R35",
  "term_label": "positive regulation of cilium assembly",
  "gene": "UniProtKB:Q8TAP8"
}